{
  "gene": "UniProtKB:P43363",
  "term_id": "GO:0042826",
  "gene_symbol": "MAGEA10",
  "gene_name": "Melanoma-associated antigen 10",
  "term_label": "histone deacetylase binding"
}